{
  "term_id": "UNKNOWN:0003",
  "gene_symbol": "FAM110A",
  "gene": "UniProtKB:Q9BQ89",
  "term_label": "Unknown cellular component",
  "gene_name": "Protein FAM110A"
}